{
  "term_id": "GO:0005615",
  "term_label": "extracellular space",
  "gene_symbol": "APOF",
  "gene_name": "Apolipoprotein F",
  "gene": "UniProtKB:Q13790"
}